{
  "term_id": "GO:0007596",
  "gene_name": "Coagulation factor XIII B chain",
  "gene": "UniProtKB:P05160",
  "term_label": "blood coagulation",
  "gene_symbol": "F13B"
}